{
  "gene": "UniProtKB:Q16720",
  "term_id": "GO:0051480",
  "gene_name": "Plasma membrane calcium-transporting ATPase 3",
  "term_label": "regulation of cytosolic calcium ion concentration",
  "gene_symbol": "ATP2B3"
}